host cell viral assembly compartment [GO:0072517] (cellular component) Relationships: is_a host intracellular membrane-bounded organelle [GO:0033648]; is a type of cytoplasmic viral factory [GO:0039714] Definition: A membrane-bounded compartment that forms in the cytoplasm of the host cell, in which virus assembly takes place. Also known as: host cell virion assembly compartment, viral assembly compartment, virion assembly compartment, host cell viral assembly site, viral assembly site References: PMID:20374631 Sources: GOC:BHF